{
  "gene_name": "Brain-specific angiogenesis inhibitor 1-associated protein 2-like protein 1",
  "gene": "UniProtKB:Q9UHR4",
  "term_label": "cytosol",
  "term_id": "GO:0005829",
  "gene_symbol": "BAIAP2L1"
}